immunoglobulin heavy chain V-D-J recombination [GO:0071707] (biological process) Definition: The process in which immunoglobulin heavy chain V, D, and J gene segments are recombined within a single locus utilizing the conserved heptamer and nonomer recombination signal sequences (RSS). Sources: GOC:add, ISBN:0781735149 Relationships: is a type of immunoglobulin V(D)J recombination [GO:0033152] Also known as: immunoglobulin V(D)J joining, immunoglobulin V(D)J recombination, immunoglobulin V-D-J joining